{
  "gene_name": "Intraflagellar transport protein 57 homolog",
  "term_label": "cilium",
  "term_id": "GO:0005929",
  "gene": "UniProtKB:Q9NWB7",
  "gene_symbol": "IFT57"
}